{
  "term_id": "GO:0030042",
  "gene": "UniProtKB:Q7RTP6",
  "gene_symbol": "MICAL3",
  "gene_name": "[F-actin]-monooxygenase MICAL3",
  "term_label": "actin filament depolymerization"
}